{
  "term_id": "GO:0005743",
  "gene": "UniProtKB:P0DKB6",
  "gene_name": "Mitochondrial pyruvate carrier 1-like protein",
  "gene_symbol": "MPC1L",
  "term_label": "mitochondrial inner membrane"
}